{
  "gene": "UniProtKB:P46939",
  "gene_symbol": "UTRN",
  "gene_name": "Utrophin",
  "term_label": "Unknown molecular function",
  "term_id": "UNKNOWN:0001"
}